{
  "term_id": "GO:0007165",
  "term_label": "signal transduction",
  "gene_symbol": "OR1E2",
  "gene_name": "Olfactory receptor 1E2",
  "gene": "UniProtKB:P47887"
}